pyrimidine deoxyribonucleoside salvage [GO:0043099] (biological process) Definition: Any process that generates a pyrimidine deoxyribonucleoside from derivatives of it, without de novo synthesis. Subtypes: deoxycytidine salvage [GO:0006237] Sources: GOC:jl Relationships: is a type of GO:0043097; is a type of GO:0046126